{
  "term_label": "Unknown molecular function",
  "gene_symbol": "PPDPF",
  "term_id": "UNKNOWN:0001",
  "gene": "UniProtKB:Q9H3Y8",
  "gene_name": "Pancreatic progenitor cell differentiation and proliferation factor"
}